{
  "term_label": "T cell activation involved in immune response",
  "gene_symbol": "IFNE",
  "gene_name": "Interferon epsilon",
  "gene": "UniProtKB:Q86WN2",
  "term_id": "GO:0002286"
}